collagenous component of basement membrane [GO:0140143] (cellular component) Relationships: is a type of external encapsulating structure [GO:0030312]; is part of GO:0140139 Definition: Collagenous component of basement membrane ECMs, including collagen IV and other types of collagen specifically expressed in basement membrane. References: PMID:21123617, PMID:21421915, PMID:28040522, PMID:28324731, PMID:31387942, PMID:39223427